L-ribulose-5-phosphate 3-epimerase activity [GO:0034015] (molecular function) Also known as: L-xylulose 5-phosphate 3-epimerase activity, SgaU, UlaE Sources: EC:5.1.3.22, RHEA:18497 Definition: Catalysis of the reaction: L-ribulose 5-phosphate = L-xylulose 5-phosphate. Relationships: is a type of GO:0016857